monounsaturated fatty acid biosynthetic process [GO:1903966] (biological process) Definition: The chemical reactions and pathways resulting in the formation of monounsaturated fatty acid. References: PMID:16443825 Sources: GOC:TermGenie, GOC:hjd, GO_REF:0000068 Also known as: monounsaturated fatty acid anabolism, monounsaturated fatty acid biosynthesis, monounsaturated fatty acid formation, monounsaturated fatty acid synthesis Note: For example, stearoyl-coenzyme A desaturase (Scd) catalyzes the desaturation of saturated fatty acids to monounsaturated fatty acids in mammals and yeast. Relationships: is a type of fatty acid biosynthetic process [GO:0006633]; is a type of monounsaturated fatty acid metabolic process [GO:1903964]